{
  "term_label": "1-phosphatidylinositol-4-phosphate 5-kinase activity",
  "gene_symbol": "PIP5KL1",
  "gene": "UniProtKB:Q5T9C9",
  "term_id": "GO:0016308",
  "gene_name": "Phosphatidylinositol 4-phosphate 5-kinase-like protein 1"
}